{
  "gene": "UniProtKB:P82932",
  "term_id": "GO:0003735",
  "term_label": "structural constituent of ribosome",
  "gene_name": "Small ribosomal subunit protein bS6m",
  "gene_symbol": "MRPS6"
}